{
  "gene": "UniProtKB:Q9BUV8",
  "gene_symbol": "RAB5IF",
  "gene_name": "GEL complex subunit OPTI",
  "term_label": "Unknown molecular function",
  "term_id": "UNKNOWN:0001"
}